{
  "term_label": "skeletal muscle tissue development",
  "term_id": "GO:0007519",
  "gene_name": "Popeye domain-containing protein 2",
  "gene": "UniProtKB:Q9HBU9",
  "gene_symbol": "POPDC2"
}